inorganic diphosphate transport [GO:0030505] (biological process) Also known as: inorganic pyrophosphate transport Sources: GOC:mah Relationships: is a type of inorganic anion transport [GO:0015698] Definition: The directed movement of inorganic diphosphate into, out of or within a cell, or between cells, by means of some agent such as a transporter or pore.